{
  "term_id": "UNKNOWN:0001",
  "gene": "UniProtKB:Q9NW08",
  "gene_symbol": "POLR3B",
  "term_label": "Unknown molecular function",
  "gene_name": "DNA-directed RNA polymerase III subunit RPC2"
}